{
  "term_id": "GO:0005634",
  "term_label": "nucleus",
  "gene_name": "Replication termination factor 2",
  "gene": "UniProtKB:Q9BY42",
  "gene_symbol": "RTF2"
}